cell growth mode switching, bipolar to monopolar [GO:0051524] (biological process) Relationships: is a type of establishment of monopolar cell polarity [GO:0061162]; is a type of regulation of direction of cell growth [GO:0061389] Sources: GOC:ai Definition: The process in which a cell switches from bipolar cell growth to monopolar cell growth.